{
  "gene_name": "Amyloid beta precursor protein binding family B member 1",
  "term_id": "GO:0006355",
  "gene_symbol": "APBB1",
  "gene": "UniProtKB:O00213",
  "term_label": "regulation of DNA-templated transcription"
}